{
  "gene": "UniProtKB:P60520",
  "gene_name": "Gamma-aminobutyric acid receptor-associated protein-like 2",
  "term_label": "autophagosome maturation",
  "gene_symbol": "GABARAPL2",
  "term_id": "GO:0097352"
}